{
  "gene_name": "Cyclin-dependent kinases regulatory subunit 2",
  "term_label": "regulation of mitotic cell cycle",
  "gene": "UniProtKB:P33552",
  "term_id": "GO:0007346",
  "gene_symbol": "CKS2"
}